{
  "gene": "UniProtKB:Q96KW2",
  "term_id": "GO:0008139",
  "term_label": "nuclear localization sequence binding",
  "gene_symbol": "POM121L2",
  "gene_name": "POM121-like protein 2"
}